{
  "term_id": "GO:0006952",
  "gene_symbol": "NOX4",
  "gene": "UniProtKB:Q9NPH5",
  "term_label": "defense response",
  "gene_name": "NADPH oxidase 4"
}